positive regulation of cellular component organization [GO:0051130] (biological process) Also known as: positive regulation of cell organisation, up regulation of cell organization, up-regulation of cell organization, upregulation of cell organization, activation of cell organization, stimulation of cell organization, positive regulation of cellular component organization and biogenesis Sources: GOC:ai Subtypes: positive regulation of organelle organization [GO:0010638], positive regulation of very-low-density lipoprotein particle remodeling [GO:0010902], positive regulation of protein-containing complex assembly [GO:0031334], positive regulation of cell projection organization [GO:0031346], positive regulation of protein-containing complex disassembly [GO:0043243], positive regulation of integrin biosynthetic process [GO:0045726], positive regulation of endocytosis [GO:0045807], positive regulation of synapse structural plasticity [GO:0051835], positive regulation of syncytium formation by plasma membrane fusion [GO:0060143], GO:0061092, positive regulation of erythrocyte enucleation [GO:0061931], GO:0090129, GO:0090261, GO:0090319, GO:0150117, positive regulation of hyaluranon cable assembly [GO:1900106], positive regulation of terminal button organization [GO:1901614], positive regulation of postsynaptic membrane organization [GO:1901628], positive regulation of presynaptic membrane organization [GO:1901631], positive regulation of synaptic vesicle membrane organization [GO:1901634], positive regulation of cell junction assembly [GO:1901890], GO:1901893, positive regulation of capsule organization [GO:1901915], positive regulation of supramolecular fiber organization [GO:1902905], GO:1903024, positive regulation of extracellular matrix organization [GO:1903055], positive regulation of vitellogenesis [GO:1903188], positive regulation of iron-sulfur cluster assembly [GO:1903331], GO:1903393, positive regulation of membrane tubulation [GO:1903527], positive regulation of plasma membrane raft polarization [GO:1903908], positive regulation of fusion of virus membrane with host plasma membrane [GO:1903915], positive regulation of neuromuscular junction development [GO:1904398], positive regulation of tight junction disassembly [GO:1905075], positive regulation of membrane invagination [GO:1905155], GO:1905559, GO:1905608, positive regulation of plasma membrane repair [GO:1905686], positive regulation of synapse pruning [GO:1905808], positive regulation of blood microparticle formation [GO:2000334], positive regulation of barbed-end actin filament capping [GO:2000814] Relationships: is a type of positive regulation of cellular process [GO:0048522]; is a type of regulation of cellular component organization [GO:0051128]; positively regulates GO:0016043 Definition: Any process that activates or increases the frequency, rate or extent of a process involved in the formation, arrangement of constituent parts, or disassembly of cell structures, including the plasma membrane and any external encapsulating structures such as the cell wall and cell envelope.